fibroblast growth factor receptor apoptotic signaling pathway [GO:1902178] (biological process) Definition: An apoptotic signaling pathway that starts with a ligand binding to, or being withdrawn from, a fibroblast growth factor receptor (FGFR). References: PMID:17561467 Sources: GOC:TermGenie, GOC:mtg_apoptosis, GOC:pm, GOC:pr Also known as: FGF receptor signaling pathway involved in apoptotic cell death, FGF receptor signaling pathway involved in apoptotic process, FGF receptor signaling pathway involved in apoptotic programmed cell death, FGF receptor signaling pathway involved in programmed cell death by apoptosis, FGF receptor signalling pathway involved in apoptotic cell death, FGF receptor signalling pathway involved in apoptotic process, FGF receptor signalling pathway involved in apoptotic programmed cell death, FGF receptor signalling pathway involved in programmed cell death by apoptosis, FGFR signaling pathway involved in apoptotic cell death, FGFR signaling pathway involved in apoptotic process, FGFR signaling pathway involved in apoptotic programmed cell death, FGFR signaling pathway involved in programmed cell death by apoptosis, fibroblast growth factor receptor signaling pathway involved in apoptotic cell death, fibroblast growth factor receptor signaling pathway involved in apoptotic process, fibroblast growth factor receptor signaling pathway involved in apoptotic programmed cell death, fibroblast growth factor receptor signaling pathway involved in programmed cell death by apoptosis, fibroblast growth factor receptor signalling pathway involved in apoptotic cell death, fibroblast growth factor receptor signalling pathway involved in apoptotic process, fibroblast growth factor receptor signalling pathway involved in apoptotic programmed cell death, fibroblast growth factor receptor signalling pathway involved in programmed cell death by apoptosis, FGF receptor signaling pathway involved in apoptosis, FGF receptor signaling pathway involved in apoptotic program, FGF receptor signaling pathway involved in type I programmed cell death, FGF receptor signalling pathway involved in apoptosis, FGF receptor signalling pathway involved in apoptotic program, FGF receptor signalling pathway involved in type I programmed cell death, FGFR signaling pathway involved in apoptosis, FGFR signaling pathway involved in apoptotic program, FGFR signaling pathway involved in type I programmed cell death, fibroblast growth factor receptor signaling pathway involved in apoptosis, fibroblast growth factor receptor signaling pathway involved in apoptotic program, fibroblast growth factor receptor signaling pathway involved in type I programmed cell death, fibroblast growth factor receptor signalling pathway involved in apoptosis, fibroblast growth factor receptor signalling pathway involved in apoptotic program, fibroblast growth factor receptor signalling pathway involved in type I programmed cell death, FGF receptor signaling pathway involved in signaling (initiator) caspase activity, FGF receptor signalling pathway involved in signaling (initiator) caspase activity, FGFR signaling pathway involved in signaling (initiator) caspase activity, fibroblast growth factor receptor signaling pathway involved in signaling (initiator) caspase activity, fibroblast growth factor receptor signalling pathway involved in signaling (initiator) caspase activity Relationships: is a type of fibroblast growth factor receptor signaling pathway [GO:0008543]; is a type of extrinsic apoptotic signaling pathway [GO:0097191]